cell competition in a multicellular organism [GO:0035212] (BP) References: PMID:1116643, PMID:15066286 Sources: GOC:bf Relationships: is a type of cellular process [GO:0009987]; is a type of regulation of growth [GO:0040008]; BFO_0000050 GO:0007275 Definition: Competitive interactions within multicellular organisms between cell populations that differ in growth rates, leading to the elimination of the slowest-growing cells.